{
  "gene_name": "Fez family zinc finger protein 2",
  "gene_symbol": "FEZF2",
  "term_id": "GO:0010468",
  "term_label": "regulation of gene expression",
  "gene": "UniProtKB:Q8TBJ5"
}